{
  "gene_symbol": "SEPTIN10",
  "gene_name": "Septin-10",
  "term_id": "GO:0032153",
  "gene": "UniProtKB:Q9P0V9",
  "term_label": "cell division site"
}